{
  "term_id": "GO:0005886",
  "gene_symbol": "GRAP",
  "term_label": "plasma membrane",
  "gene": "UniProtKB:Q13588",
  "gene_name": "GRB2-related adapter protein"
}